{
  "term_id": "GO:0035371",
  "term_label": "microtubule plus-end",
  "gene_symbol": "NCKAP5",
  "gene_name": "Nck-associated protein 5",
  "gene": "UniProtKB:O14513"
}